{
  "term_label": "Unknown cellular component",
  "gene_symbol": "ZBTB22",
  "gene_name": "Zinc finger and BTB domain-containing protein 22",
  "term_id": "UNKNOWN:0003",
  "gene": "UniProtKB:O15209"
}